{
  "term_id": "GO:0000981",
  "gene": "UniProtKB:Q8NBF1",
  "gene_name": "Zinc finger protein GLIS1",
  "term_label": "DNA-binding transcription factor activity, RNA polymerase II-specific",
  "gene_symbol": "GLIS1"
}